{
  "gene_name": "SRSF protein kinase 2",
  "term_label": "protein serine/threonine kinase activity",
  "gene": "UniProtKB:P78362",
  "gene_symbol": "SRPK2",
  "term_id": "GO:0004674"
}